{
  "gene_name": "Immunoglobulin kappa variable 3-20",
  "term_id": "GO:0006955",
  "gene": "UniProtKB:P01619",
  "gene_symbol": "IGKV3-20",
  "term_label": "immune response"
}